{
  "term_label": "positive regulation of cell population proliferation",
  "term_id": "GO:0008284",
  "gene_name": "Homeobox protein Meis3",
  "gene_symbol": "MEIS3",
  "gene": "UniProtKB:Q99687"
}